{
  "term_label": "guanyl-nucleotide exchange factor activity",
  "gene_symbol": "DEPTOR",
  "term_id": "GO:0005085",
  "gene": "UniProtKB:Q8TB45",
  "gene_name": "DEP domain-containing mTOR-interacting protein"
}